{
  "gene_symbol": "HMGN4",
  "gene_name": "High mobility group nucleosome-binding domain-containing protein 4",
  "gene": "UniProtKB:O00479",
  "term_label": "chromatin organization",
  "term_id": "GO:0006325"
}